{
  "gene": "UniProtKB:A6NLI5",
  "gene_name": "Tripartite motif-containing protein 64C",
  "term_label": "regulation of gene expression",
  "term_id": "GO:0010468",
  "gene_symbol": "TRIM64C"
}